ADP-L-glycero-beta-D-manno-heptose biosynthetic process [GO:0097171] (biological process) Definition: The chemical reactions and pathways resulting in the formation of ADP-L-glycero-beta-D-manno-heptose, an ADP-L-glycero-D-manno-heptose having beta-configuration at the anomeric centre of the heptose. ADP-L-glycero-beta-D-manno-heptose (also called ADP-L-beta-D-heptose or ADP-L-glycero-D-manno-heptose) is a nucleotide-sugar precursor of the inner core lipopolysaccharide (LPS) from D-glycero-beta-D-manno-heptose 7-phosphate. Relationships: is_a GO:0009226 Also known as: ADP-L-glycero-beta-D-manno-heptose anabolism, ADP-L-glycero-beta-D-manno-heptose biosynthesis, ADP-L-glycero-beta-D-manno-heptose formation, ADP-L-glycero-beta-D-manno-heptose synthesis References: PMID:11751812 Sources: GOC:yaf